{
  "gene": "UniProtKB:Q8TC41",
  "gene_symbol": "RNF217",
  "term_id": "GO:0006511",
  "term_label": "ubiquitin-dependent protein catabolic process",
  "gene_name": "E3 ubiquitin-protein ligase RNF217"
}